{
  "term_label": "Unknown biological process",
  "term_id": "UNKNOWN:0002",
  "gene_symbol": "SPINK8",
  "gene": "UniProtKB:P0C7L1",
  "gene_name": "Serine protease inhibitor Kazal-type 8"
}